{
  "gene_name": "Protein Wnt-7a",
  "gene": "UniProtKB:O00755",
  "term_label": "positive regulation of JNK cascade",
  "gene_symbol": "WNT7A",
  "term_id": "GO:0046330"
}